negative regulation of ATP biosynthetic process [GO:2001170] (biological process) Sources: GOC:obol Definition: Any process that stops, prevents or reduces the frequency, rate or extent of ATP biosynthetic process. Subtypes: negative regulation of mitochondrial ATP synthesis coupled proton transport [GO:1905707] Relationships: is_a GO:1900372; is a type of negative regulation of ATP metabolic process [GO:1903579]; is a type of regulation of ATP biosynthetic process [GO:2001169]; RO_0002212 ATP biosynthetic process [GO:0006754] Also known as: negative regulation of ATP anabolism, negative regulation of ATP biosynthesis, negative regulation of ATP formation, negative regulation of ATP synthesis, negative regulation of ATP regeneration